{
  "term_label": "nucleus",
  "term_id": "GO:0005634",
  "gene_symbol": "ZNF765",
  "gene_name": "Zinc finger protein 765",
  "gene": "UniProtKB:Q7L2R6"
}